{
  "gene_name": "Cilium assembly protein DZIP1L",
  "term_id": "GO:0036064",
  "gene_symbol": "DZIP1L",
  "gene": "UniProtKB:Q8IYY4",
  "term_label": "ciliary basal body"
}